{
  "gene": "UniProtKB:Q15714",
  "term_id": "GO:0008284",
  "gene_name": "TSC22 domain family protein 1",
  "gene_symbol": "TSC22D1",
  "term_label": "positive regulation of cell population proliferation"
}